{
  "gene_name": "Angiomotin",
  "gene_symbol": "AMOT",
  "gene": "UniProtKB:Q4VCS5",
  "term_id": "GO:0038023",
  "term_label": "signaling receptor activity"
}